{
  "gene_symbol": "KCNN1",
  "gene_name": "Small conductance calcium-activated potassium channel protein 1",
  "term_id": "GO:0005886",
  "gene": "UniProtKB:Q92952",
  "term_label": "plasma membrane"
}